{
  "gene_symbol": "ABHD8",
  "gene": "UniProtKB:Q96I13",
  "term_id": "GO:0055088",
  "gene_name": "Protein ABHD8",
  "term_label": "lipid homeostasis"
}